{
  "gene_symbol": "ACVRL1",
  "term_label": "cell differentiation",
  "gene_name": "Serine_threonine-protein kinase receptor R3",
  "term_id": "GO:0030154",
  "gene": "UniProtKB:P37023"
}